U6 snRNA 3'-end binding [GO:0030629] (molecular function) Definition: Binding to a U6 small nuclear RNA (U6 snRNA) at the 3' end. Sources: GOC:mah Note: Note that this term may be useful for annotating small nuclear RNAs (snRNAs). Relationships: is a type of U6 snRNA binding [GO:0017070] Also known as: U6 snRNA 3' end binding